{
  "term_id": "UNKNOWN:0003",
  "gene_name": "Putative uncharacterized protein PRO0255",
  "gene_symbol": "PRO0255",
  "term_label": "Unknown cellular component",
  "gene": "UniProtKB:Q9UI72"
}